{
  "gene": "UniProtKB:O15534",
  "gene_name": "Period circadian protein homolog 1",
  "term_id": "GO:0001222",
  "term_label": "transcription corepressor binding",
  "gene_symbol": "PER1"
}